heme metabolic process [GO:0042168] (biological process) Relationships: is a type of porphyrin-containing compound metabolic process [GO:0006778]; is a type of pigment metabolic process [GO:0042440] Also known as: haem metabolic process, haem metabolism, heme metabolism Definition: The chemical reactions and pathways involving heme, any compound of iron complexed in a porphyrin (tetrapyrrole) ring. Subtypes: GO:0006783, heme oxidation [GO:0006788], GO:0042167 Sources: GOC:jl, ISBN:0124325653